3-phosphoshikimate 1-carboxyvinyltransferase activity [GO:0003866] (molecular function) Also known as: 3-enol-pyruvoylshikimate-5-phosphate synthase activity, 5-enolpyruvylshikimate-3-phosphate synthase activity, EPSP synthase activity, phosphoenolpyruvate:3-phosphoshikimate 5-O-(1-carboxyvinyl)-transferase activity Definition: Catalysis of the reaction: 3-phosphoshikimate + phosphoenolpyruvate = 5-O-(1-carboxyvinyl)-3-phosphoshikimate + phosphate. Sources: EC:2.5.1.19, RHEA:21256 Relationships: is a type of GO:0016765